{
  "gene_name": "Huntingtin-interacting protein K",
  "term_label": "negative regulation of apoptotic process",
  "term_id": "GO:0043066",
  "gene_symbol": "HYPK",
  "gene": "UniProtKB:Q9NX55"
}